positive regulation of wound healing, spreading of epidermal cells [GO:1903691] (biological process) Also known as: up regulation of wound healing, spreading of epidermal cells, up-regulation of wound healing, spreading of epidermal cells, upregulation of wound healing, spreading of epidermal cells, activation of wound healing, spreading of epidermal cells Relationships: is a type of positive regulation of cell migration [GO:0030335]; is a type of positive regulation of wound healing [GO:0090303]; is a type of GO:1903689; positively regulates wound healing, spreading of epidermal cells [GO:0035313] Definition: Any process that activates or increases the frequency, rate or extent of wound healing, spreading of epidermal cells. References: PMID:18394891 Sources: GOC:TermGenie, GOC:als, GO_REF:0000058